positive regulation of filamentous growth of a population of unicellular organisms in response to pH [GO:1900743] (BP) Definition: Any process that activates or increases the frequency, rate or extent of filamentous growth of a population of unicellular organisms in response to pH. Sources: GOC:TermGenie, GOC:di Subtypes: GO:1900442 Relationships: is a type of GO:0048584; is a type of positive regulation of filamentous growth of a population of unicellular organisms [GO:1900430]; is a type of regulation of filamentous growth of a population of unicellular organisms in response to pH [GO:1900741]; positively regulates filamentous growth of a population of unicellular organisms in response to pH [GO:0036177] Also known as: up regulation of filamentous growth of a population of unicellular organisms in response to pH, up-regulation of filamentous growth of a population of unicellular organisms in response to pH, upregulation of filamentous growth of a population of unicellular organisms in response to pH, activation of filamentous growth of a population of unicellular organisms in response to pH